{
  "gene": "UniProtKB:Q14790",
  "gene_symbol": "CASP8",
  "term_id": "GO:0008625",
  "gene_name": "Caspase-8",
  "term_label": "extrinsic apoptotic signaling pathway via death domain receptors"
}